{
  "gene_symbol": "EP300",
  "term_label": "histone acetyltransferase activity",
  "gene_name": "Histone acetyltransferase p300",
  "term_id": "GO:0004402",
  "gene": "UniProtKB:Q09472"
}